regulation of toll-like receptor 10 signaling pathway [GO:0034167] (biological process) Also known as: regulation of TLR10 signaling pathway, regulation of toll-like receptor 10 signalling pathway References: PMID:16551253, PMID:17328678 Sources: GOC:add Subtypes: negative regulation of toll-like receptor 10 signaling pathway [GO:0034168], positive regulation of toll-like receptor 10 signaling pathway [GO:0034169] Definition: Any process that modulates the frequency, rate, or extent of toll-like receptor 10 signaling pathway. Relationships: is a type of regulation of pattern recognition receptor signaling pathway [GO:0062207]; regulates toll-like receptor 10 signaling pathway [GO:0034166]